{
  "term_label": "plasma membrane",
  "gene_name": "Glycerophosphodiester phosphodiesterase 1",
  "term_id": "GO:0005886",
  "gene_symbol": "GDE1",
  "gene": "UniProtKB:Q9NZC3"
}